{
  "gene": "UniProtKB:Q56NI9",
  "gene_symbol": "ESCO2",
  "gene_name": "N-acetyltransferase ESCO2",
  "term_id": "GO:0000785",
  "term_label": "chromatin"
}